{
  "term_label": "RNA polymerase II cis-regulatory region sequence-specific DNA binding",
  "gene_symbol": "HES5",
  "term_id": "GO:0000978",
  "gene_name": "Transcription factor HES-5",
  "gene": "UniProtKB:Q5TA89"
}